{
  "gene_name": "Long-chain fatty acid transport protein 2",
  "gene_symbol": "SLC27A2",
  "term_label": "peroxisomal membrane",
  "term_id": "GO:0005778",
  "gene": "UniProtKB:O14975"
}